{
  "gene_name": "Putative transmembrane protein INAFM2",
  "term_label": "Unknown cellular component",
  "gene_symbol": "INAFM2",
  "term_id": "UNKNOWN:0003",
  "gene": "UniProtKB:P0DMQ5"
}